{
  "gene_name": "Ubiquitin domain-containing protein UBFD1",
  "gene_symbol": "UBFD1",
  "gene": "UniProtKB:O14562",
  "term_id": "UNKNOWN:0003",
  "term_label": "Unknown cellular component"
}